{
  "term_id": "GO:0005829",
  "gene": "UniProtKB:Q9UI26",
  "term_label": "cytosol",
  "gene_symbol": "IPO11",
  "gene_name": "Importin-11"
}